{
  "term_label": "RNA processing",
  "term_id": "GO:0006396",
  "gene": "UniProtKB:Q8WTP8",
  "gene_symbol": "AEN",
  "gene_name": "Apoptosis-enhancing nuclease"
}